maintenance of inflorescence meristem identity [GO:0010077] (biological process) Definition: The process in which an organism retains a population of inflorescence meristem cells, preventing the commitment of all stem cell progeny to a differentiated cell fate. Sources: GOC:dph, GOC:tb Relationships: is a type of maintenance of meristem identity [GO:0010074]